{
  "gene_symbol": "PTGER1",
  "term_label": "prostaglandin E receptor activity",
  "gene_name": "Prostaglandin E2 receptor EP1 subtype",
  "term_id": "GO:0004957",
  "gene": "UniProtKB:P34995"
}